{
  "gene_name": "E3 ubiquitin-protein ligase ARIH1",
  "gene": "UniProtKB:Q9Y4X5",
  "term_id": "GO:0031624",
  "term_label": "ubiquitin conjugating enzyme binding",
  "gene_symbol": "ARIH1"
}